{
  "term_label": "actin filament fragmentation",
  "gene_name": "Cofilin-1",
  "term_id": "GO:0030043",
  "gene_symbol": "CFL1",
  "gene": "UniProtKB:P23528"
}